indole glucosinolate catabolic process [GO:0042344] (biological process) Relationships: is a type of glucosinolate catabolic process [GO:0019762]; is a type of GO:0042343; is a type of indole-containing compound catabolic process [GO:0042436] Also known as: indole glucosinolate breakdown, indole glucosinolate catabolism, indole glucosinolate degradation Definition: The chemical reactions and pathways resulting in the breakdown of indole glucosinolates, sulfur-containing compounds that have a common structure linked to an R group derived from tryptophan. References: PMID:29122987